{
  "gene_symbol": "MED17",
  "term_label": "mediator complex",
  "gene_name": "Mediator of RNA polymerase II transcription subunit 17",
  "term_id": "GO:0016592",
  "gene": "UniProtKB:Q9NVC6"
}